arachidonate metabolic process [GO:0019369] (BP) Subtypes: cyclooxygenase pathway [GO:0019371], epoxygenase P450 pathway [GO:0019373], omega-hydroxylase P450 pathway [GO:0097267] Relationships: is a type of long-chain fatty acid metabolic process [GO:0001676]; is a type of GO:0006690; is a type of unsaturated fatty acid metabolic process [GO:0033559]; is_a olefinic compound metabolic process [GO:0120254] Sources: ISBN:0198506732 Definition: The chemical reactions and pathways involving arachidonic acid, a straight chain fatty acid with 20 carbon atoms and four double bonds per molecule. Arachidonic acid is the all-Z-(5,8,11,14)-isomer. Also known as: arachidonic acid metabolic process, arachidonic acid metabolism